fructose catabolic process [GO:0006001] (biological process) Also known as: fructose breakdown, fructose catabolism, fructose degradation Definition: The chemical reactions and pathways resulting in the breakdown of fructose, the ketohexose arabino-2-hexulose. Sources: GOC:ai Relationships: is a type of GO:0006000; is a type of hexose catabolic process [GO:0019320] Subtypes: GO:0061616, fructose catabolic process to hydroxyacetone phosphate and glyceraldehyde-3-phosphate [GO:0061624], GO:0061625